{
  "gene_symbol": "ACSM2B",
  "gene_name": "Acyl-coenzyme A synthetase ACSM2B, mitochondrial",
  "term_label": "fatty-acyl-CoA synthase activity",
  "term_id": "GO:0004321",
  "gene": "UniProtKB:Q68CK6"
}